{
  "term_label": "plasma membrane",
  "term_id": "GO:0005886",
  "gene": "UniProtKB:Q16281",
  "gene_symbol": "CNGA3",
  "gene_name": "Cyclic nucleotide-gated cation channel alpha-3"
}